carboxyvinyl-carboxyphosphonate phosphorylmutase activity [GO:0008807] (molecular function) Also known as: 1-carboxyvinyl carboxyphosphonate phosphorylmutase (decarboxylating), CPEP phosphonomutase activity, carboxyphosphonoenolpyruvate phosphonomutase activity Definition: Catalysis of the reaction: 1-carboxyvinyl carboxyphosphonate = 3-(hydrohydroxyphosphoryl)pyruvate + CO2. Relationships: is a type of GO:0016780 Sources: EC:2.7.8.23